{
  "term_label": "Unknown cellular component",
  "term_id": "UNKNOWN:0003",
  "gene": "UniProtKB:Q9H4I3",
  "gene_symbol": "TRABD",
  "gene_name": "TraB domain-containing protein"
}